{
  "gene_symbol": "HLA-DOB",
  "term_label": "late endosome membrane",
  "gene_name": "HLA class II histocompatibility antigen, DO beta chain",
  "term_id": "GO:0031902",
  "gene": "UniProtKB:P13765"
}